type 1 neuromedin U receptor binding [GO:0031839] (MF) Also known as: type 1 neuromedin U receptor ligand Sources: GOC:mah, GOC:nln Relationships: is a type of neuromedin U receptor binding [GO:0042922] Definition: Binding to a type 1 neuromedin U receptor.